positive regulation of mesenchymal cell proliferation involved in lung development [GO:2000792] (biological process) Relationships: is a type of positive regulation of mesenchymal cell proliferation [GO:0002053]; is a type of positive regulation of developmental process [GO:0051094]; is a type of positive regulation of multicellular organismal process [GO:0051240]; is a type of GO:2000790; positively regulates mesenchymal cell proliferation involved in lung development [GO:0060916] References: PMID:21513708 Definition: Any process that activates or increases the frequency, rate or extent of mesenchymal cell proliferation involved in lung development.